N(omega)-methyl-L-arginine catabolic process [GO:2001297] (biological process) Definition: The chemical reactions and pathways resulting in the breakdown of N(omega)-methyl-L-arginine. References: PMID:10510241 Sources: GOC:rs Also known as: N(omega)-methyl-L-arginine breakdown, N(omega)-methyl-L-arginine catabolism, N(omega)-methyl-L-arginine degradation Relationships: is_a GO:0042219; is a type of GO:0170035; is a type of non-proteinogenic amino acid catabolic process [GO:0170044]